{
  "gene_symbol": "COL3A1",
  "term_id": "GO:0005586",
  "gene": "UniProtKB:P02461",
  "term_label": "collagen type III trimer",
  "gene_name": "Collagen alpha-1(III) chain"
}